{
  "term_label": "membrane",
  "gene_symbol": "OR12D1",
  "gene": "UniProtKB:P0DN82",
  "gene_name": "Olfactory receptor 12D1",
  "term_id": "GO:0016020"
}